{
  "gene_symbol": "HS3ST6",
  "term_label": "Unknown biological process",
  "gene": "UniProtKB:Q96QI5",
  "gene_name": "Heparan sulfate glucosamine 3-O-sulfotransferase 6",
  "term_id": "UNKNOWN:0002"
}